{
  "term_label": "RNA polymerase II general transcription initiation factor activity",
  "gene": "UniProtKB:Q8IZX4",
  "gene_symbol": "TAF1L",
  "gene_name": "Transcription initiation factor TFIID subunit 1-like",
  "term_id": "GO:0016251"
}